actin filament debranching [GO:0071846] (biological process) Relationships: is a type of actin filament severing [GO:0051014] Definition: An actin filament severing process that results in the removal of actin filament branches specifically at the branch points. References: PMID:20362448 Sources: GOC:jh, GOC:mah